{
  "gene_symbol": "MUC22",
  "term_id": "UNKNOWN:0003",
  "gene": "UniProtKB:E2RYF6",
  "term_label": "Unknown cellular component",
  "gene_name": "Mucin-22"
}